{
  "term_id": "GO:0007064",
  "gene_symbol": "PDS5A",
  "gene": "UniProtKB:Q29RF7",
  "gene_name": "Sister chromatid cohesion protein PDS5 homolog A",
  "term_label": "mitotic sister chromatid cohesion"
}